{
  "gene_name": "Iroquois-class homeodomain protein IRX-1",
  "gene_symbol": "IRX1",
  "term_label": "RNA polymerase II cis-regulatory region sequence-specific DNA binding",
  "term_id": "GO:0000978",
  "gene": "UniProtKB:P78414"
}